negative regulation of erythrocyte clearance [GO:0034107] (biological process) Relationships: is a type of negative regulation of immune system process [GO:0002683]; is_a GO:0034104; is a type of regulation of erythrocyte clearance [GO:0034106]; negatively regulates erythrocyte clearance [GO:0034102] References: PMID:12905029, PMID:14754397 Sources: GOC:add Also known as: negative regulation of RBC clearance, negative regulation of red blood cell clearance, negative regulation of neocytolysis Definition: Any process that stops, prevents, or reduces the frequency, rate, or extent of erythrocyte clearance.